phenylethylamine catabolic process [GO:0019607] (biological process) Definition: The chemical reactions and pathways resulting in the breakdown of phenylethylamine, an amine with pharmacological properties similar to those of amphetamine, occurs naturally as a neurotransmitter in the brain, and is present in chocolate and oil of bitter almonds. Sources: GOC:jl, ISBN:0395825172 Also known as: phenylethylamine breakdown, phenylethylamine catabolism, phenylethylamine degradation Relationships: is a type of biogenic amine catabolic process [GO:0042402]; is a type of phenylethylamine metabolic process [GO:0042443]; is a type of primary amino compound catabolic process [GO:1901161]